{
  "gene_symbol": "GPS1",
  "gene": "UniProtKB:Q13098",
  "term_label": "Unknown molecular function",
  "gene_name": "COP9 signalosome complex subunit 1",
  "term_id": "UNKNOWN:0001"
}